{
  "gene_symbol": "SHMT2",
  "term_id": "GO:0046653",
  "term_label": "tetrahydrofolate metabolic process",
  "gene": "UniProtKB:P34897",
  "gene_name": "Serine hydroxymethyltransferase, mitochondrial"
}